{
  "gene_symbol": "H3-3B",
  "term_label": "structural constituent of chromatin",
  "term_id": "GO:0030527",
  "gene_name": "Histone H3.3",
  "gene": "UniProtKB:P84243"
}